{
  "term_id": "GO:0016831",
  "gene_name": "Acidic amino acid decarboxylase GADL1",
  "term_label": "carboxy-lyase activity",
  "gene": "UniProtKB:Q6ZQY3",
  "gene_symbol": "GADL1"
}